isopentenyl diphosphate biosynthetic process [GO:0009240] (biological process) Relationships: is a type of phospholipid biosynthetic process [GO:0008654]; is a type of isopentenyl diphosphate metabolic process [GO:0046490]; is part of isoprenoid biosynthetic process [GO:0008299] Also known as: IPP biosynthesis, IPP biosynthetic process, isopentenyl diphosphate anabolism, isopentenyl diphosphate biosynthesis, isopentenyl diphosphate formation, isopentenyl diphosphate synthesis, isopentenyl pyrophosphate biosynthesis, isopentenyl pyrophosphate biosynthetic process Definition: The chemical reactions and pathways resulting in the formation of isopentenyl diphosphate, an isomer of dimethylallyl diphosphate and the key precursor of all isoprenoids. Subtypes: isopentenyl diphosphate biosynthetic process, mevalonate pathway [GO:0019287], GO:0019288 Sources: GOC:jl, ISBN:0198506732